{
  "term_label": "dihydrofolate metabolic process",
  "gene_name": "Dihydrofolate reductase 2, mitochondrial",
  "gene_symbol": "DHFR2",
  "gene": "UniProtKB:Q86XF0",
  "term_id": "GO:0046452"
}